CDP-glycerol diphosphatase activity [GO:0047734] (molecular function) Definition: Catalysis of the reaction: CDP-glycerol + H2O = sn-glycerol 3-phosphate + CMP + 2 H+. Sources: EC:3.6.1.16, RHEA:21692 Also known as: CDP-glycerol pyrophosphatase activity, CDP-glycerol phosphoglycerohydrolase activity, CDPglycerol diphosphatase activity, CDPglycerol phosphoglycerohydrolase activity, CDPglycerol pyrophosphatase activity, cytidine diphosphoglycerol pyrophosphatase activity Relationships: is a type of pyrophosphatase activity [GO:0016462]